{
  "gene": "UniProtKB:Q9H3P2",
  "gene_symbol": "NELFA",
  "gene_name": "Negative elongation factor A",
  "term_label": "negative regulation of transcription elongation by RNA polymerase II",
  "term_id": "GO:0034244"
}